{
  "gene_name": "Vacuolar protein sorting-associated protein 29",
  "gene": "UniProtKB:Q9UBQ0",
  "gene_symbol": "VPS29",
  "term_label": "retromer complex",
  "term_id": "GO:0030904"
}